ether catabolic process [GO:1901502] (biological process) Subtypes: 6-hydroxycineole catabolic process [GO:0019639], GO:0036040, vanillin catabolic process [GO:0042190], GO:0042856, glycerol ether catabolic process [GO:0044269], 2,4,5-trichlorophenoxyacetic acid catabolic process [GO:0046228], 2,4-dichlorophenoxyacetic acid catabolic process [GO:0046300], diorcinol catabolic process [GO:1900571], gerfelin catabolic process [GO:1900577], violaceol I catabolic process [GO:1900589], violaceol II catabolic process [GO:1900592], emericellin catabolic process [GO:1900765], fonsecin catabolic process [GO:1900768], cordyol C catabolic process [GO:1900798], ferulate catabolic process [GO:1901067], spheroidene catabolic process [GO:1901179], GO:1901511, GO:1901752, GO:1901779, 1,5-anhydro-D-fructose catabolic process [GO:1901802], GO:1901832, GO:1902085, (-)-pinoresinol catabolic process [GO:1902123], (+)-pinoresinol catabolic process [GO:1902125], GO:1902131 Relationships: is a type of catabolic process [GO:0009056] Definition: The chemical reactions and pathways resulting in the breakdown of ether. Also known as: ether breakdown, ether catabolism, ether degradation Sources: GOC:TermGenie, GOC:pr